{
  "gene_name": "Interleukin-4 receptor subunit alpha",
  "term_label": "external side of plasma membrane",
  "gene_symbol": "IL4R",
  "term_id": "GO:0009897",
  "gene": "UniProtKB:P24394"
}